{
  "gene": "UniProtKB:Q32P44",
  "term_id": "GO:0072686",
  "term_label": "mitotic spindle",
  "gene_symbol": "EML3",
  "gene_name": "Echinoderm microtubule-associated protein-like 3"
}